{
  "gene": "UniProtKB:P42857",
  "gene_symbol": "NSG1",
  "term_id": "GO:0032051",
  "term_label": "clathrin light chain binding",
  "gene_name": "Neuronal vesicle trafficking-associated protein 1"
}